deoxycytidylate 5-hydroxymethyltransferase activity [GO:0047153] (molecular function) Sources: EC:2.1.2.8, RHEA:11280 Relationships: is a type of GO:0016742 Also known as: deoxycytidylate hydroxymethyltransferase activity, 5,10-methylenetetrahydrofolate:deoxycytidylate 5-hydroxymethyltransferase activity, d-cytidine 5'-monophosphate hydroxymethylase activity, dCMP hydroxymethylase activity, deoxyCMP hydroxymethylase activity, deoxycytidylate hydroxymethylase activity, deoxycytidylic hydroxymethylase activity Definition: Catalysis of the reaction: 5,10-methylenetetrahydrofolate + dCMP + H2O = (6S)-5,6,7,8-tetrahydrofolate + 5-hydroxymethyldeoxycytidylate.